regulation of exocyst localization [GO:0060178] (biological process) Relationships: is a type of regulation of localization [GO:0032879]; regulates exocyst localization [GO:0051601] Definition: Any process that modulates the localization of exocysts. An exocyst is a protein complex peripherally associated with the plasma membrane that determines where vesicles dock and fuse. Also known as: regulation of exocyst localisation Sources: GOC:dph, GOC:tb